Rac protein signal transduction [GO:0016601] (biological process) Relationships: is a type of small GTPase-mediated signal transduction [GO:0007264] Also known as: Rac mediated signal transduction Regulation: regulated by regulation of Rac protein signal transduction [GO:0035020]; negatively regulated by negative regulation of Rac protein signal transduction [GO:0035021]; positively regulated by positive regulation of Rac protein signal transduction [GO:0035022] Sources: GOC:bf Definition: An intracellular signaling cassette in which a small monomeric GTPase of the Rac subfamily relays a signal.